{
  "gene": "UniProtKB:O96011",
  "gene_symbol": "PEX11B",
  "term_label": "peroxisomal membrane",
  "gene_name": "Peroxisomal membrane protein 11B",
  "term_id": "GO:0005778"
}